{
  "gene": "UniProtKB:Q9NP99",
  "gene_symbol": "TREM1",
  "term_id": "GO:0009986",
  "term_label": "cell surface",
  "gene_name": "Triggering receptor expressed on myeloid cells 1"
}